{
  "term_label": "Unknown biological process",
  "gene_symbol": "FANCD2OS",
  "gene_name": "FANCD2 opposite strand protein",
  "gene": "UniProtKB:Q96PS1",
  "term_id": "UNKNOWN:0002"
}